{
  "gene": "UniProtKB:P35249",
  "gene_symbol": "RFC4",
  "term_id": "GO:0005663",
  "gene_name": "Replication factor C subunit 4",
  "term_label": "DNA replication factor C complex"
}